respiratory chain complex IV [GO:0045277] (cellular component) Relationships: is a type of GO:0070069; is a type of respiratory chain complex [GO:0098803]; is a type of GO:1902495 Also known as: cytochrome c oxidase complex, electron transport complex IV Definition: A part of the respiratory chain, containing the 13 polypeptide subunits of cytochrome c oxidase, including cytochrome a and cytochrome a3. Catalyzes the oxidation of reduced cytochrome c by dioxygen (O2). Sources: ISBN:0198547684